GTP cyclohydrolase II activity [GO:0003935] (molecular function) Sources: EC:3.5.4.25, RHEA:23704 Definition: Catalysis of the reaction: GTP + 4 H2O = 2,5-diamino-6-hydroxy-4-(5-phosphoribosylamino)-pyrimidine + formate + 3 H+ + 2 phosphate. Also known as: GTP 7,8-8,9-dihydrolase (diphosphate-forming), GTP-8-formylhydrolase activity, guanosine triphosphate cyclohydrolase II Relationships: is a type of GTP cyclohydrolase activity [GO:0003933]